{
  "term_id": "UNKNOWN:0003",
  "term_label": "Unknown cellular component",
  "gene_symbol": "RELT",
  "gene": "UniProtKB:Q969Z4",
  "gene_name": "Tumor necrosis factor receptor superfamily member 19L"
}